{
  "term_id": "GO:0016324",
  "gene_name": "Transient receptor potential cation channel subfamily M member 6",
  "gene": "UniProtKB:Q9BX84",
  "gene_symbol": "TRPM6",
  "term_label": "apical plasma membrane"
}